{
  "gene_symbol": "OR2G2",
  "gene_name": "Olfactory receptor 2G2",
  "gene": "UniProtKB:Q8NGZ5",
  "term_id": "GO:0050911",
  "term_label": "detection of chemical stimulus involved in sensory perception of smell"
}